fumonisin biosynthetic process [GO:1900541] (biological process) Sources: GOC:TermGenie Also known as: fumonisin anabolism, fumonisin biosynthesis, fumonisin formation, fumonisin synthesis Definition: The chemical reactions and pathways resulting in the formation of fumonisin. Relationships: is a type of secondary metabolite biosynthetic process [GO:0044550]; is a type of GO:0046394 Regulation: regulated by regulation of fumonisin biosynthetic process [GO:1900683]; negatively regulated by GO:1900684; positively regulated by positive regulation of fumonisin biosynthetic process [GO:1900685]